{
  "term_id": "UNKNOWN:0002",
  "gene": "UniProtKB:O95825",
  "gene_symbol": "CRYZL1",
  "term_label": "Unknown biological process",
  "gene_name": "Quinone oxidoreductase-like protein 1"
}